{
  "gene_symbol": "INPP5B",
  "term_label": "membrane",
  "term_id": "GO:0016020",
  "gene": "UniProtKB:P32019",
  "gene_name": "Type II inositol 1,4,5-trisphosphate 5-phosphatase"
}